{
  "term_label": "Unknown biological process",
  "term_id": "UNKNOWN:0002",
  "gene_symbol": "ANKRD33B",
  "gene": "UniProtKB:A6NCL7",
  "gene_name": "Ankyrin repeat domain-containing protein 33B"
}